{
  "gene_symbol": "ALMS1",
  "term_label": "regulation of centriole replication",
  "gene_name": "Centrosome-associated protein ALMS1",
  "gene": "UniProtKB:Q8TCU4",
  "term_id": "GO:0046599"
}